{
  "term_label": "chemical synaptic transmission",
  "gene_symbol": "HRH4",
  "gene": "UniProtKB:Q9H3N8",
  "gene_name": "Histamine H4 receptor",
  "term_id": "GO:0007268"
}